{
  "term_label": "sprouting angiogenesis",
  "gene": "UniProtKB:P35916",
  "gene_name": "Vascular endothelial growth factor receptor 3",
  "gene_symbol": "FLT4",
  "term_id": "GO:0002040"
}